pellicle [GO:0020039] (cellular component) Relationships: is a type of GO:0110165 Definition: The structure enclosing certain parasite cells such as certain apicomplexa and Euglenozoa; consists of the cell membrane with its associated infrastructure of microtubules, microfilaments and other organelles. Sources: GOC:mah, GOC:mb